{
  "gene": "UniProtKB:Q15388",
  "gene_name": "Mitochondrial import receptor subunit TOM20 homolog",
  "term_id": "GO:0008320",
  "term_label": "protein transmembrane transporter activity",
  "gene_symbol": "TOMM20"
}